{
  "gene": "UniProtKB:P0C091",
  "term_label": "cell-matrix adhesion",
  "gene_name": "FRAS1-related extracellular matrix protein 3",
  "term_id": "GO:0007160",
  "gene_symbol": "FREM3"
}